{
  "gene": "UniProtKB:A4FU28",
  "term_label": "endoplasmic reticulum exit site",
  "gene_symbol": "CTAGE9",
  "gene_name": "cTAGE family member 9",
  "term_id": "GO:0070971"
}